{
  "term_label": "Unknown cellular component",
  "gene": "UniProtKB:Q8N8D7",
  "term_id": "UNKNOWN:0003",
  "gene_name": "Sodium_potassium-transporting ATPase subunit beta-1-interacting protein 3",
  "gene_symbol": "NKAIN3"
}